{
  "gene_symbol": "IRX3",
  "gene": "UniProtKB:P78415",
  "term_label": "neuron differentiation",
  "term_id": "GO:0030182",
  "gene_name": "Iroquois-class homeodomain protein IRX-3"
}